{
  "term_label": "double-stranded telomeric DNA binding",
  "gene": "UniProtKB:Q92878",
  "gene_name": "DNA repair protein RAD50",
  "gene_symbol": "RAD50",
  "term_id": "GO:0003691"
}